{
  "gene": "UniProtKB:Q6UUV9",
  "term_label": "positive regulation of transcription by RNA polymerase II",
  "gene_symbol": "CRTC1",
  "gene_name": "CREB-regulated transcription coactivator 1",
  "term_id": "GO:0045944"
}